{
  "gene": "UniProtKB:Q16082",
  "term_id": "GO:0005737",
  "gene_name": "Heat shock protein beta-2",
  "term_label": "cytoplasm",
  "gene_symbol": "HSPB2"
}